Se-methyltransferase activity [GO:0051995] (molecular function) Relationships: is a type of methyltransferase activity [GO:0008168] Subtypes: selenocysteine methyltransferase activity [GO:0016205] Sources: GOC:ai Definition: Catalysis of the transfer of a methyl group to the selenium atom of an acceptor molecule.